{
  "term_id": "UNKNOWN:0001",
  "gene_symbol": "USP27X",
  "term_label": "Unknown molecular function",
  "gene_name": "Ubiquitin carboxyl-terminal hydrolase 27",
  "gene": "UniProtKB:A6NNY8"
}